{
  "gene_name": "Protein FAM228B",
  "gene_symbol": "FAM228B",
  "term_id": "UNKNOWN:0003",
  "term_label": "Unknown cellular component",
  "gene": "UniProtKB:P0C875"
}